{
  "gene_name": "Intracellular hyaluronan-binding protein 4",
  "term_label": "cytoplasm",
  "gene": "UniProtKB:Q5JVS0",
  "gene_symbol": "HABP4",
  "term_id": "GO:0005737"
}